histone H3 methyltransferase activity [GO:0140938] (molecular function) Definition: Catalysis of the reaction: S-adenosyl-L-methionine + a histone H3 = S-adenosyl-L-homocysteine + a methylated histone H3. Histone methylation generally occurs on either an arginine or a lysine residue. Also known as: histone H3 methylase activity, histone H3 methylation Relationships: is_a histone methyltransferase activity [GO:0042054] References: PMID:28450737 Subtypes: histone H3K79 methyltransferase activity [GO:0031151], histone H3R17 methyltransferase activity [GO:0035642], histone H3K4 methyltransferase activity [GO:0042800], histone H3K9 methyltransferase activity [GO:0046974], GO:0046975, GO:0046976, GO:0062122, histone H3R2 methyltransferase activity [GO:0070611], histone H3R8 methyltransferase activity [GO:0140592], histone H3K56 methyltransferase activity [GO:0140759], histone H3R26 methyltransferase activity [GO:0140903]